{
  "gene_name": "Interferon-inducible protein AIM2",
  "gene": "UniProtKB:O14862",
  "gene_symbol": "AIM2",
  "term_id": "GO:0097169",
  "term_label": "AIM2 inflammasome complex"
}